{
  "gene_name": "Cell adhesion molecule 2",
  "term_id": "GO:0007156",
  "term_label": "homophilic cell-cell adhesion",
  "gene": "UniProtKB:Q8N3J6",
  "gene_symbol": "CADM2"
}